protein urmylation [GO:0032447] (biological process) Relationships: is a type of protein modification by small protein conjugation [GO:0032446] Definition: Covalent attachment of the ubiquitin-like protein URM1 to another protein. Sources: GOC:vw